gallate dioxygenase activity [GO:0036238] (molecular function) Relationships: is a type of oxidoreductase activity, acting on single donors with incorporation of molecular oxygen, incorporation of two atoms of oxygen [GO:0016702] References: PMID:16030014 Sources: EC:1.13.11.57 Definition: Catalysis of the reaction: gallate + O2 = (1E)-4-oxobut-1-ene-1,2,4-tricarboxylate.